{
  "gene": "UniProtKB:Q96PU5",
  "term_id": "GO:0050807",
  "gene_symbol": "NEDD4L",
  "term_label": "regulation of synapse organization",
  "gene_name": "E3 ubiquitin-protein ligase NEDD4-like"
}